{
  "term_id": "GO:0005737",
  "gene_name": "Cyclin-dependent kinase 4 inhibitor B",
  "gene_symbol": "CDKN2B",
  "gene": "UniProtKB:P42772",
  "term_label": "cytoplasm"
}